{
  "term_id": "GO:0005737",
  "term_label": "cytoplasm",
  "gene_symbol": "RELB",
  "gene": "UniProtKB:Q01201",
  "gene_name": "Transcription factor RelB"
}